urease complex [GO:0035550] (cellular component) Definition: A multiprotein nickel-containing complex that possesses urease activity (catalysis of the hydrolysis of urea to ammonia and carbon dioxide). Relationships: is a type of catalytic complex [GO:1902494]; is part of cytoplasm [GO:0005737] Note: Eukaryotic microorganisms, plants, and probably Gram-positive bacteria, possess a homopolymeric urease. In contrast, urease complexes from gram-negative bacteria studied thus far clearly possess three distinct subunits (alpha, beta and gamma). Tightly bound nickel is present in all urease complexes. References: PMID:2651866 Sources: InterPro:IPR008221